{
  "gene_name": "UPF0547 protein C16orf87",
  "term_id": "UNKNOWN:0003",
  "gene_symbol": "C16orf87",
  "gene": "UniProtKB:Q6PH81",
  "term_label": "Unknown cellular component"
}